{
  "gene_symbol": "HBS1L",
  "term_label": "GTPase activity",
  "gene_name": "HBS1-like protein",
  "gene": "UniProtKB:Q9Y450",
  "term_id": "GO:0003924"
}